UDP-glucuronate 5'-epimerase activity [GO:0050379] (molecular function) Sources: GOC:curators Also known as: UDP-glucuronate 5' epimerase activity, C-5-uronosyl epimerase activity, UDP-glucuronic acid 5'-epimerase activity, UDP-glucuronic acid epimerase activity, UDPglucuronate 5'-epimerase activity, uridine diphosphoglucuronate 5'-epimerase activity Definition: Catalysis of the reaction: UDP-alpha-D-glucuronate = UDP-L-iduronate. Relationships: is a type of racemase and epimerase activity, acting on carbohydrates and derivatives [GO:0016857]